cellular response to catecholamine stimulus [GO:0071870] (biological process) Subtypes: cellular response to norepinephrine stimulus [GO:0071874], cellular response to dopamine [GO:1903351], cellular response to oxidopamine [GO:1905842] Sources: GOC:BHF, GOC:mah Definition: Any process that results in a change in state or activity of a cell (in terms of movement, secretion, enzyme production, gene expression, etc.) as a result of a catecholamine stimulus. A catecholamine is any of a group of biogenic amines that includes 4-(2-aminoethyl)pyrocatechol [4-(2-aminoethyl)benzene-1,2-diol] and derivatives formed by substitution. Relationships: is_a cellular response to monoamine stimulus [GO:0071868]; is a type of response to catecholamine [GO:0071869]; is_a cellular response to oxygen-containing compound [GO:1901701]